{
  "gene_symbol": "OR5V1",
  "gene": "UniProtKB:Q9UGF6",
  "term_id": "GO:0004984",
  "gene_name": "Olfactory receptor 5V1",
  "term_label": "olfactory receptor activity"
}